{
  "term_id": "GO:0000122",
  "term_label": "negative regulation of transcription by RNA polymerase II",
  "gene_name": "LIM domain-binding protein 1",
  "gene_symbol": "LDB1",
  "gene": "UniProtKB:Q86U70"
}